regulation of mesenchymal cell apoptotic process involved in metanephros development [GO:1900211] (biological process) Subtypes: regulation of mesenchymal cell apoptotic process involved in metanephric nephron morphogenesis [GO:0072304], negative regulation of mesenchymal cell apoptotic process involved in metanephros development [GO:1900212], positive regulation of mesenchymal cell apoptotic process involved in metanephros development [GO:1900213] References: PMID:17314325 Sources: GOC:TermGenie, GOC:mtg_apoptosis, GOC:mtg_kidney_jan10, GOC:yaf Also known as: regulation of mesenchymal cell apoptosis involved in metanephros development Definition: Any process that modulates the frequency, rate or extent of mesenchymal cell apoptotic process involved in metanephros development. Relationships: is a type of regulation of apoptotic process involved in development [GO:1904748]; is a type of regulation of mesenchymal cell apoptotic process [GO:2001053]; regulates mesenchymal cell apoptotic process involved in metanephros development [GO:1900200]